{
  "gene_symbol": "CYP1A1",
  "gene": "UniProtKB:P04798",
  "term_id": "GO:0008395",
  "term_label": "steroid hydroxylase activity",
  "gene_name": "Cytochrome P450 1A1"
}